L-alanine oxidation to D-lactate and ammonia [GO:0019479] (biological process) Sources: MetaCyc:ALACAT2-PWY Relationships: is a type of L-alanine catabolic process [GO:0042853] Definition: The chemical reactions and pathways resulting in the breakdown of L-alanine to D-lactate and ammonia.